{
  "gene_symbol": "PHOSPHO1",
  "gene": "UniProtKB:Q8TCT1",
  "term_id": "GO:0035630",
  "gene_name": "Phosphoethanolamine_phosphocholine phosphatase",
  "term_label": "bone mineralization involved in bone maturation"
}